{
  "gene_symbol": "NCOR1",
  "term_label": "nuclear thyroid hormone receptor binding",
  "gene": "UniProtKB:O75376",
  "term_id": "GO:0046966",
  "gene_name": "Nuclear receptor corepressor 1"
}